sinoatrial node cell development [GO:0060931] (biological process) Relationships: is a type of cardiac pacemaker cell development [GO:0060926]; is part of GO:0060921 Sources: GOC:mtg_heart Also known as: SA node cell development, SAN cell development, sinus node cell development Definition: The process whose specific outcome is the progression of a sinoatrial (SA) node cell over time, from its formation to the mature state. SA node cells are pacemaker cells that are found in the sinoatrial node.